lysine transport [GO:0015819] (BP) Subtypes: L-lysine transmembrane import into vacuole [GO:0090517] Sources: GOC:ai Definition: The directed movement of lysine, 2,6-diaminohexanoic acid, into, out of or within a cell, or between cells, by means of some agent such as a transporter or pore. Also known as: L-lysine import, lysine import, lysine uptake, L-lysine transport Relationships: is a type of basic amino acid transport [GO:0015802]; is a type of GO:1902022